{
  "gene": "UniProtKB:Q6NSW5",
  "gene_name": "Putative DENN domain-containing protein 10 B",
  "term_label": "regulation of early endosome to late endosome transport",
  "term_id": "GO:2000641",
  "gene_symbol": "DENND10P1"
}